{
  "term_id": "GO:0005759",
  "gene_name": "Alpha-ketoglutarate-dependent dioxygenase alkB homolog 7, mitochondrial",
  "term_label": "mitochondrial matrix",
  "gene": "UniProtKB:Q9BT30",
  "gene_symbol": "ALKBH7"
}